{
  "gene_symbol": "RAB6A",
  "term_label": "retrograde transport, endosome to Golgi",
  "gene": "UniProtKB:P20340",
  "gene_name": "Ras-related protein Rab-6A",
  "term_id": "GO:0042147"
}